regulation of protein geranylgeranylation [GO:2000539] (biological process) Also known as: regulation of protein amino acid geranylgeranylation, regulation of C-terminal protein geranylgeranylation Relationships: is a type of regulation of macromolecule biosynthetic process [GO:0010556]; is_a regulation of protein modification process [GO:0031399]; regulates protein geranylgeranylation [GO:0018344] Definition: Any process that modulates the frequency, rate or extent of protein geranylgeranylation. Sources: GOC:obol Subtypes: negative regulation of protein geranylgeranylation [GO:2000540], GO:2000541